archaeosine-tRNA biosynthetic process [GO:0002927] (biological process) Note: Archaeosine (7-formamidino-7-deazaguanosine) is a structural variant of the hypermodified nucleoside 7-deazaguanosine. The biosynthesis pathway starts with archaeosine tRNA-guanine transglycosylase (ArcTGT) which catalyzes the exchange of guanine at position 15 in the D-loop of archaeal tRNAs with a free 7-cyano-7-deazaguanine. Relationships: is a type of tRNA modification [GO:0006400]; is a type of biosynthetic process [GO:0009058]; has part archaeosine synthase activity [GO:0002948]; has part GO:0043867 References: PMID:20129918 Sources: GOC:hjd Definition: The chemical reactions and pathways involved in the biosynthesis of archaeosine, an archaea-specific modified base found at position 15 in the D-loop of certain archaeal tRNAs.